{
  "gene_symbol": "GON7",
  "term_label": "EKC/KEOPS complex",
  "gene_name": "EKC_KEOPS complex subunit GON7",
  "term_id": "GO:0000408",
  "gene": "UniProtKB:Q9BXV9"
}